kinetochore disassembly [GO:0062096] (biological process) Definition: The disaggregation of a kinetochore into its constituent components. References: PMID:27611693 Sources: GOC:mah Relationships: is a type of GO:0051383; is a type of organelle disassembly [GO:1903008]